{
  "term_label": "defense response to Gram-positive bacterium",
  "gene_name": "Beta-defensin 1",
  "term_id": "GO:0050830",
  "gene": "UniProtKB:P60022",
  "gene_symbol": "DEFB1"
}